{
  "gene": "UniProtKB:Q96EH5",
  "term_id": "GO:0002181",
  "gene_name": "Ribosomal protein eL39-like 2",
  "gene_symbol": "RPL39L",
  "term_label": "cytoplasmic translation"
}